{
  "term_label": "nucleus",
  "term_id": "GO:0005634",
  "gene": "UniProtKB:Q6ZNG1",
  "gene_name": "Zinc finger protein 600",
  "gene_symbol": "ZNF600"
}